{
  "gene_symbol": "SLC27A2",
  "term_label": "long-chain fatty acid transmembrane transporter activity",
  "term_id": "GO:0005324",
  "gene": "UniProtKB:O14975",
  "gene_name": "Long-chain fatty acid transport protein 2"
}